zeaxanthin bis(beta-D-glucoside) biosynthetic process [GO:1901830] (biological process) Relationships: is a type of GO:0016117; is a type of beta-glucoside biosynthetic process [GO:1901806] Also known as: zeaxanthin bis(beta-D-glucoside) anabolism, zeaxanthin bis(beta-D-glucoside) biosynthesis, zeaxanthin bis(beta-D-glucoside) formation, zeaxanthin bis(beta-D-glucoside) synthesis, zeaxanthin diglucoside anabolism, zeaxanthin diglucoside biosynthesis, zeaxanthin diglucoside formation, zeaxanthin diglucoside synthesis References: PMID:20075616 Sources: GOC:TermGenie, GOC:yaf, MetaCyc:PWY-6288, UniPathway:UPA00798 Definition: The chemical reactions and pathways resulting in the formation of zeaxanthin bis(beta-D-glucoside).